D-amino-acid N-acetyltransferase activity [GO:0047812] (molecular function) Sources: RHEA:20704 Subtypes: D-tryptophan N-acetyltransferase activity [GO:0047835] Relationships: is a type of GO:0008080 Definition: Catalysis of the reaction: acetyl-CoA + a D-amino acid = CoA + an N-acetyl-D-amino-acid. Also known as: D-amino acid acetyltransferase activity, D-amino acid-alpha-N-acetyltransferase activity, acetyl-CoA:D-amino-acid N-acetyltransferase activity